{
  "term_id": "GO:0030424",
  "gene_symbol": "CNTN1",
  "gene": "UniProtKB:Q12860",
  "gene_name": "Contactin-1",
  "term_label": "axon"
}